{
  "gene_name": "Nuclear factor of activated T-cells, cytoplasmic 1",
  "term_id": "GO:0000978",
  "gene_symbol": "NFATC1",
  "term_label": "RNA polymerase II cis-regulatory region sequence-specific DNA binding",
  "gene": "UniProtKB:O95644"
}